{
  "gene_symbol": "IRF3",
  "gene": "UniProtKB:Q14653",
  "term_id": "GO:0005634",
  "gene_name": "Interferon regulatory factor 3",
  "term_label": "nucleus"
}